{
  "gene_name": "Actin-like protein 8",
  "gene_symbol": "ACTL8",
  "term_id": "GO:0048870",
  "term_label": "cell motility",
  "gene": "UniProtKB:Q9H568"
}